signal transduction in absence of ligand [GO:0038034] (biological process) Subtypes: ligand-independent adenylate cyclase-activating G protein-coupled receptor signaling pathway [GO:0038035], GO:0097192 Definition: The series of molecular signals initiated by the absence of a ligand or the withdrawal of a ligand from a receptor. Regulation: negatively regulated by negative regulation of signal transduction in absence of ligand [GO:1901099] References: PMID:15044679 Sources: GOC:al, GOC:ppm, GOC:pr Also known as: addiction receptor signaling pathway, dependence receptor signaling pathway, non-classical signal transduction, signal transduction in absence of agonist, basal signaling, negative signal transduction Relationships: is_a signal transduction [GO:0007165]